{
  "term_id": "UNKNOWN:0001",
  "gene_symbol": "NAV1",
  "gene": "UniProtKB:Q8NEY1",
  "gene_name": "Neuron navigator 1",
  "term_label": "Unknown molecular function"
}